response to cytochalasin B [GO:1901328] (biological process) Definition: Any process that results in a change in state or activity of a cell or an organism (in terms of movement, secretion, enzyme production, gene expression, etc.) as a result of a cytochalasin B stimulus. Sources: GOC:TermGenie Relationships: is a type of response to nitrogen compound [GO:1901698]; is a type of GO:1901700 Subtypes: GO:0072749